{
  "gene_symbol": "PLEKHG4",
  "gene_name": "Puratrophin-1",
  "gene": "UniProtKB:Q58EX7",
  "term_id": "GO:0019898",
  "term_label": "extrinsic component of membrane"
}